{
  "term_id": "GO:0090263",
  "gene": "UniProtKB:Q2MKA7",
  "term_label": "positive regulation of canonical Wnt signaling pathway",
  "gene_symbol": "RSPO1",
  "gene_name": "R-spondin-1"
}